regulation of skeletal muscle contraction via regulation of action potential [GO:0014861] (biological process) Definition: Any process that modulates the frequency, rate or extent of skeletal muscle contraction by depolarization of muscle membrane and ionic fluxes. Sources: GOC:BHF, GOC:mtg_cardiac_conduct_nov11, GOC:mtg_muscle Also known as: regulation of skeletal muscle contraction via membrane action potential Relationships: is a type of GO:0014819; is_a GO:0098900; regulates regulation of skeletal muscle contraction by action potential [GO:0100001]